poly(beta-D-mannuronate) lyase activity [GO:0045135] (molecular function) Definition: Catalysis of the reaction: polysaccharides containing beta-D-mannuronate residues = oligosaccharides with 4-deoxy-alpha-L-erythro-hex-4-enopyranuronosyl end. This reaction is the eliminative cleavage of polysaccharides containing beta-D-mannuronate residues to give oligosaccharides with 4-deoxy-alpha-L-erythro-hex-4-enopyranuronosyl groups at their ends. Sources: EC:4.2.2.3 Also known as: alginate lyase I activity, poly(mana) alginate lyase activity, alginase I, alginase activity, alginate lyase activity, poly(beta-D-1,4-mannuronide) lyase activity Relationships: is_a carbon-oxygen lyase activity, acting on polysaccharides [GO:0016837]